diaminohydroxyphosphoribosylaminopyrimidine deaminase activity [GO:0008835] (molecular function) Definition: Catalysis of the reaction: 2,5-diamino-6-hydroxy-4-(5-phosphoribosylamino)-pyrimidine + H2O + H+ = 5-amino-6-(5-phosphoribosylamino)uracil + NH4. References: PMID:11889103 Sources: EC:3.5.4.26, RHEA:21868 Relationships: is a type of GO:0016814; is a type of deaminase activity [GO:0019239] Also known as: 2,5-diamino-6-(ribosylamino)-4(3H)-pyrimidinone 5'-phosphate deaminase activity, 2,5-diamino-6-hydroxy-4-(5-phosphoribosylamino)-pyrimidine 2-aminohydrolase activity, 2,5-diamino-6-hydroxy-4-(5-phosphoribosylamino)pyrimidine 2-aminohydrolase activity